{
  "term_id": "UNKNOWN:0002",
  "gene": "UniProtKB:A6NJU9",
  "gene_name": "Nuclear pore complex-interacting protein family member B13",
  "term_label": "Unknown biological process",
  "gene_symbol": "NPIPB13"
}